{
  "term_label": "Unknown molecular function",
  "term_id": "UNKNOWN:0001",
  "gene": "UniProtKB:A0A0B4J237",
  "gene_symbol": "TRAV8-2",
  "gene_name": "T cell receptor alpha variable 8-2"
}